{
  "term_id": "GO:0034431",
  "gene": "UniProtKB:O95989",
  "term_label": "bis(5'-adenosyl)-hexaphosphatase activity",
  "gene_name": "Diphosphoinositol polyphosphate phosphohydrolase 1",
  "gene_symbol": "NUDT3"
}